{
  "gene_symbol": "TOP2B",
  "gene_name": "DNA topoisomerase 2-beta",
  "term_id": "GO:0005634",
  "gene": "UniProtKB:Q02880",
  "term_label": "nucleus"
}